{
  "gene_name": "Corticotropin-releasing factor-binding protein",
  "term_label": "extracellular space",
  "gene": "UniProtKB:P24387",
  "term_id": "GO:0005615",
  "gene_symbol": "CRHBP"
}